phenylalkylamine binding [GO:0008145] (molecular function) Relationships: is a type of GO:0043176 Definition: Binding to phenylalkylamine or one of its derivatives. Sources: GOC:jl